dioxotetrahydropyrimidine phosphoribosyltransferase activity [GO:0047281] (molecular function) Definition: Catalysis of the reaction: pyrophosphate + a 2,4-dioxotetrahydropyrimidine D-ribonucleotide = PRPP + a 2,4-dioxotetrahydropyrimidine. Also known as: 2,4-dioxotetrahydropyrimidine-nucleotide:diphosphate phospho-alpha-D-ribosyltransferase activity, dioxotetrahydropyrimidine phosphoribosyl transferase activity, dioxotetrahydropyrimidine ribonucleotide pyrophosphorylase activity, dioxotetrahydropyrimidine-ribonucleotide diphosphorylase activity, dioxotetrahydropyrimidine-ribonucleotide pyrophosphorylase activity Relationships: is a type of pentosyltransferase activity [GO:0016763] Sources: EC:2.4.2.20, MetaCyc:2.4.2.20-RXN